{
  "gene_symbol": "SPANXN2",
  "gene_name": "Sperm protein associated with the nucleus on the X chromosome N2",
  "term_id": "UNKNOWN:0002",
  "gene": "UniProtKB:Q5MJ10",
  "term_label": "Unknown biological process"
}